{
  "gene_name": "Dynein light chain roadblock-type 2",
  "term_id": "GO:0005813",
  "term_label": "centrosome",
  "gene_symbol": "DYNLRB2",
  "gene": "UniProtKB:Q8TF09"
}